{
  "term_label": "Unknown cellular component",
  "term_id": "UNKNOWN:0003",
  "gene_name": "T cell receptor beta joining 1-4",
  "gene": "UniProtKB:A0A0J9YXG5",
  "gene_symbol": "TRBJ1-4"
}